{
  "gene_name": "Methylosome protein WDR77",
  "term_id": "GO:0034709",
  "gene": "UniProtKB:Q9BQA1",
  "gene_symbol": "WDR77",
  "term_label": "methylosome"
}